(+)-borneol dehydrogenase activity [GO:0047500] (molecular function) Definition: Catalysis of the reaction: (+)-borneol + NAD+ = (1R, 4R)-camphor + H+ + NADH. Sources: RHEA:17329 Also known as: (+)-borneol:NAD+ oxidoreductase activity, bicyclic monoterpenol dehydrogenase activity Relationships: is a type of oxidoreductase activity, acting on the CH-OH group of donors, NAD or NADP as acceptor [GO:0016616]; is part of (+)-camphor biosynthetic process [GO:0046211]